{
  "gene_symbol": "LGALS9",
  "term_label": "nucleus",
  "term_id": "GO:0005634",
  "gene_name": "Galectin-9",
  "gene": "UniProtKB:O00182"
}